{
  "term_id": "UNKNOWN:0001",
  "gene": "UniProtKB:Q2M329",
  "gene_name": "Coiled-coil domain-containing protein 96",
  "gene_symbol": "CFAP184",
  "term_label": "Unknown molecular function"
}